{
  "term_label": "regulation of transcription by RNA polymerase II",
  "gene": "UniProtKB:P52742",
  "gene_symbol": "ZNF135",
  "term_id": "GO:0006357",
  "gene_name": "Zinc finger protein 135"
}